{
  "term_id": "UNKNOWN:0001",
  "gene_name": "Protein JTB",
  "gene_symbol": "JTB",
  "term_label": "Unknown molecular function",
  "gene": "UniProtKB:O76095"
}